{
  "gene": "UniProtKB:P41229",
  "gene_name": "Lysine-specific demethylase 5C",
  "term_label": "chromatin remodeling",
  "term_id": "GO:0006338",
  "gene_symbol": "KDM5C"
}